neurogenesis [GO:0022008] (biological process) Sources: GOC:cls, GOC:curators, GOC:dgh, GOC:dph, GOC:jid Subtypes: gliogenesis [GO:0042063], generation of neurons [GO:0048699] Definition: Generation of cells within the nervous system. Regulation: regulated by GO:0050767; negatively regulated by negative regulation of neurogenesis [GO:0050768]; positively regulated by GO:0050769 Relationships: is a type of cell differentiation [GO:0030154]; is part of nervous system development [GO:0007399] Also known as: nervous system cell generation, neural cell differentiation